{
  "gene": "UniProtKB:Q9HBY0",
  "gene_name": "NADPH oxidase 3",
  "term_id": "GO:0006952",
  "gene_symbol": "NOX3",
  "term_label": "defense response"
}